{
  "term_label": "signaling receptor activity",
  "gene_name": "Leucine-rich repeat and immunoglobulin-like domain-containing nogo receptor-interacting protein 2",
  "gene_symbol": "LINGO2",
  "gene": "UniProtKB:Q7L985",
  "term_id": "GO:0038023"
}